{
  "gene_symbol": "FAM27D1",
  "gene_name": "Protein FAM27D1",
  "term_id": "UNKNOWN:0002",
  "gene": "UniProtKB:Q5T7N8",
  "term_label": "Unknown biological process"
}